{
  "term_label": "cytoplasm",
  "gene": "UniProtKB:Q9NZN4",
  "gene_symbol": "EHD2",
  "gene_name": "EH domain-containing protein 2",
  "term_id": "GO:0005737"
}